L-lysine catabolic process to glutarate, by acetylation [GO:0019473] (biological process) Definition: The chemical reactions and pathways resulting in the breakdown of L-lysine into other compounds, including glutarate, by acetylation. Relationships: is a type of L-lysine catabolic process [GO:0019477] Sources: GOC:go_curators Also known as: L-lysine breakdown to glutarate, by acetylation, L-lysine degradation to glutarate, by acetylation